parallel actin filament bundle [GO:0097518] (cellular component) Subtypes: formin-nucleated actin cable [GO:0070648], GO:0098859 Relationships: is a type of actin filament bundle [GO:0032432] Sources: GOC:cjm, GOC:mah, ISBN:0815316194 Definition: An actin filament bundle in which the filaments are tightly packed (approximately 10-20 nm apart) and oriented with the same polarity.